{
  "term_label": "postsynaptic intermediate filament cytoskeleton",
  "gene": "UniProtKB:P07196",
  "gene_symbol": "NEFL",
  "gene_name": "Neurofilament light polypeptide",
  "term_id": "GO:0099160"
}